corazonin receptor activity [GO:0035237] (molecular function) Relationships: is a type of GO:0008188 Definition: Combining with the neuropeptide corazonin to initiate a change in cell activity. Sources: GOC:bf